{
  "term_id": "GO:0000977",
  "gene_name": "Endothelial PAS domain-containing protein 1",
  "term_label": "RNA polymerase II transcription regulatory region sequence-specific DNA binding",
  "gene": "UniProtKB:Q99814",
  "gene_symbol": "EPAS1"
}